{
  "gene": "UniProtKB:Q8NEA9",
  "gene_name": "Germ cell-less protein-like 2",
  "term_label": "Unknown biological process",
  "term_id": "UNKNOWN:0002",
  "gene_symbol": "GMCL2"
}